venom-mediated inhibition of voltage-gated sodium channel activity [GO:0044493] (biological process) Definition: A process in which an organism inhibits or disrupts the activity of a voltage-gated sodium channel in another organism via the action of a venom. References: PMID:21781281 Sources: GOC:fj, GOC:jl Also known as: envenomation resulting in negative regulation of voltage-gated sodium channel activity in another organism, envenomation resulting in negative regulation of voltage-gated sodium channel activity in other organism Relationships: is_a venom-mediated perturbation of voltage-gated sodium channel activity [GO:0044492]